{
  "term_id": "UNKNOWN:0002",
  "term_label": "Unknown biological process",
  "gene_name": "Probable mitochondrial glutathione transporter SLC25A39",
  "gene_symbol": "SLC25A39",
  "gene": "UniProtKB:Q9BZJ4"
}